{
  "gene_symbol": "SCRIB",
  "term_id": "GO:0098609",
  "term_label": "cell-cell adhesion",
  "gene": "UniProtKB:Q14160",
  "gene_name": "Protein scribble homolog"
}